{
  "term_id": "UNKNOWN:0003",
  "term_label": "Unknown cellular component",
  "gene_name": "Uncharacterized protein",
  "gene_symbol": "A0A8Q3WLD3",
  "gene": "UniProtKB:A0A8Q3WLD3"
}